{
  "term_id": "GO:0005634",
  "gene_symbol": "NGRN",
  "gene_name": "Neugrin",
  "gene": "UniProtKB:Q9NPE2",
  "term_label": "nucleus"
}